anaerobic toluene biosynthetic process [GO:0046253] (biological process) Note: This term was reinstated from obsolete. Definition: The chemical reactions and pathways resulting in the formation of toluene, a volatile monoaromatic hydrocarbon found in crude petroleum and petroleum products, in the absence of oxygen. Also known as: anaerobic toluene anabolism, anaerobic toluene biosynthesis, anaerobic toluene formation, anaerobic toluene synthesis Relationships: is a type of GO:0046252 References: PMID:8573493 Sources: GOC:ai